{
  "term_id": "UNKNOWN:0003",
  "term_label": "Unknown cellular component",
  "gene_name": "Putative transcript Y 10 protein",
  "gene_symbol": "TTTY10",
  "gene": "UniProtKB:Q9BZA0"
}